{
  "gene_symbol": "ADAT2",
  "gene_name": "tRNA-specific adenosine deaminase 2",
  "term_id": "GO:0002100",
  "gene": "UniProtKB:Q7Z6V5",
  "term_label": "tRNA wobble adenosine to inosine editing"
}